comma-shaped body morphogenesis [GO:0072049] (biological process) Subtypes: mesonephric comma-shaped body morphogenesis [GO:0061236], metanephric comma-shaped body morphogenesis [GO:0072278] Definition: The process in which the comma-shaped body is generated and organized. The comma-shaped body is the precursor structure to the S-shaped body that contributes to the morphogenesis of the nephron. Sources: GOC:mtg_kidney_jan10 Relationships: is a type of anatomical structure morphogenesis [GO:0009653]; is part of GO:0072028